{
  "term_id": "GO:1901911",
  "term_label": "adenosine 5'-(hexahydrogen pentaphosphate) catabolic process",
  "gene": "UniProtKB:Q9NZJ9",
  "gene_name": "Diphosphoinositol polyphosphate phosphohydrolase 2",
  "gene_symbol": "NUDT4"
}